{
  "gene_name": "Putative uncharacterized protein IBA57-DT",
  "term_label": "Unknown molecular function",
  "gene_symbol": "IBA57-DT",
  "gene": "UniProtKB:B1ANH7",
  "term_id": "UNKNOWN:0001"
}